TIM23 mitochondrial import inner membrane translocase complex [GO:0005744] (cellular component) References: PMID:27554484, PMID:8851659 Relationships: is a type of GO:0098800 Also known as: mitochondrial inner membrane translocase complex, Tim23 complex, mitochondrial inner membrane pre-sequence translocase complex, mitochondrial inner membrane presequence translocase complex Definition: The protein transport machinery of the mitochondrial inner membrane that typically transports proteins that possess a matrix-targeting N-terminal presequence. The TIM23 complex contains three essential Tim proteins: Tim17 and Tim23 are thought to build a preprotein translocation channel while Tim44 interacts transiently with the matrix heat-shock protein Hsp70 to form an ATP-driven import motor. Note: See also the cellular component term 'mitochondrial inner membrane ; GO:0005743'.